{
  "gene": "UniProtKB:Q8WWT9",
  "term_label": "plasma membrane",
  "gene_name": "Na(+)_dicarboxylate cotransporter 3",
  "gene_symbol": "SLC13A3",
  "term_id": "GO:0005886"
}